{
  "term_label": "ATPase-coupled intramembrane lipid transporter activity",
  "gene_symbol": "ATP10B",
  "gene_name": "Phospholipid-transporting ATPase VB",
  "gene": "UniProtKB:O94823",
  "term_id": "GO:0140326"
}